{
  "gene_name": "Ubiquitin-conjugating enzyme E2 J1",
  "gene": "UniProtKB:Q9Y385",
  "term_label": "nucleus",
  "term_id": "GO:0005634",
  "gene_symbol": "UBE2J1"
}